tRNA(Ser) (uridine(44)-2'-O-)-methyltransferase activity [GO:0141101] (molecular function) Definition: Catalysis of the reaction: Catalysis of the reaction: S-adenosyl-L-methionine + uridine44 in tRNASer = 2'-O-methyluridine44 in tRNASer + H+ + S-adenosyl-L-homocysteine. Relationships: is a type of tRNA (uridine) methyltransferase activity [GO:0016300] References: PMID:18025252 Sources: RHEA:43100 Also known as: tRNA(Ser) (uracil(44)-2'-O-)-methyltransferase activity